ubiquitin-like protein-specific endopeptidase activity [GO:0070137] (MF) Subtypes: SUMO-specific endopeptidase activity [GO:0070139] Definition: Catalysis of the hydrolysis of peptide bonds between an alpha-carboxyl group and an alpha-amino group within a small protein such as ubiquitin or a ubiquitin-like protein (e.g. APG8, ISG15, NEDD8, SUMO). Also known as: small conjugating protein-specific endopeptidase activity Relationships: is a type of GO:0004197; is a type of ubiquitin-like protein peptidase activity [GO:0019783] Sources: GOC:mah